{
  "term_label": "mitochondrial inner membrane",
  "gene": "UniProtKB:Q9BUP0",
  "gene_symbol": "EFHD1",
  "term_id": "GO:0005743",
  "gene_name": "EF-hand domain-containing protein D1"
}